{
  "term_id": "GO:0005886",
  "gene_symbol": "LRIG2",
  "gene": "UniProtKB:O94898",
  "gene_name": "Leucine-rich repeats and immunoglobulin-like domains protein 2",
  "term_label": "plasma membrane"
}